{
  "term_label": "plasma membrane",
  "term_id": "GO:0005886",
  "gene": "UniProtKB:Q9Y6M4",
  "gene_name": "Casein kinase I isoform gamma-3",
  "gene_symbol": "CSNK1G3"
}